{
  "term_id": "GO:0005783",
  "term_label": "endoplasmic reticulum",
  "gene_symbol": "CERS2",
  "gene": "UniProtKB:Q96G23",
  "gene_name": "Ceramide synthase 2"
}